{
  "term_id": "UNKNOWN:0001",
  "gene": "UniProtKB:B4DH59",
  "gene_symbol": "NBPF26",
  "term_label": "Unknown molecular function",
  "gene_name": "Neuroblastoma breakpoint family member 26"
}